{
  "term_id": "GO:0005615",
  "gene_name": "C-C motif chemokine 3-like 1",
  "term_label": "extracellular space",
  "gene_symbol": "CCL3L1",
  "gene": "UniProtKB:P16619"
}